{
  "gene_name": "DNA replication licensing factor MCM4",
  "gene": "UniProtKB:P33991",
  "term_label": "mitotic DNA replication initiation",
  "gene_symbol": "MCM4",
  "term_id": "GO:1902975"
}